{
  "term_id": "GO:0016493",
  "gene_name": "Atypical chemokine receptor 4",
  "gene": "UniProtKB:Q9NPB9",
  "gene_symbol": "ACKR4",
  "term_label": "C-C chemokine receptor activity"
}